{
  "gene_symbol": "ZBTB34",
  "term_id": "GO:0000122",
  "gene": "UniProtKB:Q8NCN2",
  "gene_name": "Zinc finger and BTB domain-containing protein 34",
  "term_label": "negative regulation of transcription by RNA polymerase II"
}